CMP metabolic process [GO:0046035] (biological process) Relationships: is a type of pyrimidine ribonucleoside monophosphate metabolic process [GO:0009173]; is a type of pyrimidine ribonucleotide metabolic process [GO:0009218] Sources: GOC:go_curators Definition: The chemical reactions and pathways involving CMP, cytidine monophosphate. Subtypes: GO:0006248, GO:0009224 Also known as: CMP metabolism